{
  "term_id": "UNKNOWN:0002",
  "gene": "UniProtKB:Q8IX95",
  "gene_symbol": "CTAGE3P",
  "term_label": "Unknown biological process",
  "gene_name": "Putative cTAGE family member 3"
}